{
  "gene_symbol": "PIERCE2",
  "gene": "UniProtKB:H3BRN8",
  "gene_name": "Piercer of microtubule wall 2 protein",
  "term_id": "UNKNOWN:0001",
  "term_label": "Unknown molecular function"
}